{
  "term_label": "protein polyubiquitination",
  "term_id": "GO:0000209",
  "gene": "UniProtKB:Q9Y6I7",
  "gene_name": "WD repeat and SOCS box-containing protein 1",
  "gene_symbol": "WSB1"
}